histone H3K9 methyltransferase activity [GO:0046974] (molecular function) Note: Comment: Note that the residue position corresponds to the canonical human H3 histone (UniProtKB:P84243); this residue is conserved across all eukaryotes. Residue 1 is the first residue following removal of the initiating Methionine (Met). Note that each histone is encoded by multiple genes, and sequences may vary across different genes within an organism. Also known as: histone H3K9 methylase activity, histone lysine N-methyltransferase activity (H3-K9 specific), histone methylase activity (H3-K9 specific), histone methyltransferase activity (H3-K9 specific), histone-H3K9 methyltransferase activity Sources: GOC:ai Subtypes: histone H3K9 dimethyltransferase activity [GO:0140942], GO:0140947, GO:0140948, histone H3K9 trimethyltransferase activity [GO:0140949] Definition: Catalysis of the reaction: S-adenosyl-L-methionine + histone H3 L-lysine (position 9) = S-adenosyl-L-homocysteine + histone H3 N6-methyl-L-lysine (position 9). This reaction is the addition of up to three methyl groups to the lysine residue at position 9 of the histone H3 protein. Relationships: is a type of protein-lysine N-methyltransferase activity [GO:0016279]; is a type of histone H3 methyltransferase activity [GO:0140938]